histone H2A kinase activity [GO:0140995] (molecular function) References: PMID:25303536 Relationships: is a type of histone kinase activity [GO:0035173] Subtypes: GO:0044024, histone H2AT120 kinase activity [GO:1990244] Definition: Catalysis of the transfer of a phosphate group to a histone H2A.